chrysanthemyl diphosphate synthase activity [GO:0033849] (molecular function) Relationships: is a type of GO:0016765 Also known as: CPPase activity, dimethylallyl-diphosphate:dimethylallyl-diphosphate dimethylallyltransferase (chrysanthemyl-diphosphate-forming) activity Sources: EC:2.5.1.67, RHEA:14009 Definition: Catalysis of the reaction: 2 dimethylallyl diphosphate = (R,R)-chrysanthemyl diphosphate + diphosphate.